{
  "gene_symbol": "MATCAP1",
  "term_label": "Unknown molecular function",
  "gene_name": "Microtubule-associated tyrosine carboxypeptidase 1",
  "term_id": "UNKNOWN:0001",
  "gene": "UniProtKB:Q68EN5"
}